{
  "gene_symbol": "USP35",
  "term_id": "GO:0005634",
  "gene_name": "Ubiquitin carboxyl-terminal hydrolase 35",
  "term_label": "nucleus",
  "gene": "UniProtKB:Q9P2H5"
}